cardiac pacemaker cell development [GO:0060926] (biological process) Sources: GOC:mtg_cardiac_conduct_nov11, GOC:mtg_heart Definition: The process whose specific outcome is the progression of a pacemaker cell over time, from its formation to the mature state. Pacemaker cells are specialized cardiomyocytes that are responsible for regulating the timing of heart contractions. Subtypes: GO:0060928, sinoatrial node cell development [GO:0060931] Relationships: is a type of cardiac muscle cell development [GO:0055013]; is part of cardiac pacemaker cell differentiation [GO:0060920] Also known as: pacemaker cell development